{
  "gene_name": "Putative protein FAM74A3",
  "term_id": "UNKNOWN:0003",
  "gene": "UniProtKB:Q4VXF1",
  "term_label": "Unknown cellular component",
  "gene_symbol": "FAM74A3"
}